{
  "term_label": "Unknown biological process",
  "gene_name": "Small G protein signaling modulator 3",
  "gene": "UniProtKB:Q96HU1",
  "gene_symbol": "SGSM3",
  "term_id": "UNKNOWN:0002"
}